{
  "gene_symbol": "ABHD12B",
  "gene": "UniProtKB:Q7Z5M8",
  "term_label": "monoacylglycerol lipase activity",
  "term_id": "GO:0047372",
  "gene_name": "Protein ABHD12B"
}